{
  "term_label": "protein kinase activator activity",
  "term_id": "GO:0030295",
  "gene_symbol": "MOB1B",
  "gene_name": "MOB kinase activator 1B",
  "gene": "UniProtKB:Q7L9L4"
}